tatiopterin biosynthetic process [GO:1900870] (biological process) Definition: The chemical reactions and pathways resulting in the formation of tatiopterin. Sources: GOC:TermGenie, GOC:mengo_curators Relationships: is a type of GO:0042559; is a type of carboxylic acid biosynthetic process [GO:0046394]; is a type of GO:1900869 Also known as: tatiopterin anabolism, tatiopterin biosynthesis, tatiopterin formation, tatiopterin synthesis Regulation: regulated by regulation of tatiopterin biosynthetic process [GO:1900974]; negatively regulated by negative regulation of tatiopterin biosynthetic process [GO:1900975]; positively regulated by positive regulation of tatiopterin biosynthetic process [GO:1900976]